demethylkotanin biosynthetic process [GO:1900599] (biological process) Also known as: demethylkotanin anabolism, demethylkotanin biosynthesis, demethylkotanin formation, demethylkotanin synthesis Relationships: is a type of secondary metabolite biosynthetic process [GO:0044550] Regulation: regulated by regulation of demethylkotanin biosynthetic process [GO:1900652]; negatively regulated by negative regulation of demethylkotanin biosynthetic process [GO:1900653]; positively regulated by positive regulation of demethylkotanin biosynthetic process [GO:1900654] Definition: The chemical reactions and pathways resulting in the formation of demethylkotanin. Sources: GOC:TermGenie, GOC:di